{
  "term_id": "UNKNOWN:0002",
  "gene": "UniProtKB:Q9Y4M8",
  "gene_name": "Putative uncharacterized protein encoded by LINC00588",
  "term_label": "Unknown biological process",
  "gene_symbol": "LINC00588"
}